{
  "gene_name": "E3 UFM1-protein ligase 1",
  "gene": "UniProtKB:O94874",
  "term_label": "reticulophagy",
  "term_id": "GO:0061709",
  "gene_symbol": "UFL1"
}